{
  "gene_name": "Uncharacterized protein C16orf95",
  "gene_symbol": "C16orf95",
  "term_id": "UNKNOWN:0001",
  "term_label": "Unknown molecular function",
  "gene": "UniProtKB:Q9H693"
}